{
  "term_id": "GO:0019901",
  "gene_name": "POTE ankyrin domain family member J",
  "gene_symbol": "POTEJ",
  "term_label": "protein kinase binding",
  "gene": "UniProtKB:P0CG39"
}